{
  "term_label": "arachidonate metabolic process",
  "gene_name": "Polyunsaturated fatty acid lipoxygenase ALOX15B",
  "term_id": "GO:0019369",
  "gene": "UniProtKB:O15296",
  "gene_symbol": "ALOX15B"
}